{
  "gene_name": "Protocadherin alpha-8",
  "term_id": "GO:0050839",
  "gene_symbol": "PCDHA8",
  "gene": "UniProtKB:Q9Y5H6",
  "term_label": "cell adhesion molecule binding"
}